{
  "term_id": "GO:0005829",
  "gene_name": "TSC22 domain family protein 1",
  "gene_symbol": "TSC22D1",
  "gene": "UniProtKB:Q15714",
  "term_label": "cytosol"
}